{
  "gene": "UniProtKB:P23258",
  "gene_symbol": "TUBG1",
  "term_id": "GO:0007020",
  "term_label": "microtubule nucleation",
  "gene_name": "Tubulin gamma-1 chain"
}